{
  "term_id": "GO:0042824",
  "gene_symbol": "TAP1",
  "gene_name": "Antigen peptide transporter 1",
  "term_label": "MHC class I peptide loading complex",
  "gene": "UniProtKB:Q03518"
}